{
  "term_label": "Unknown cellular component",
  "gene": "UniProtKB:Q5VV17",
  "gene_name": "OTU domain-containing protein 1",
  "gene_symbol": "OTUD1",
  "term_id": "UNKNOWN:0003"
}